{
  "gene_name": "Arylsulfatase G",
  "term_id": "UNKNOWN:0002",
  "gene_symbol": "ARSG",
  "term_label": "Unknown biological process",
  "gene": "UniProtKB:Q96EG1"
}